{
  "term_label": "focal adhesion",
  "gene_name": "Paxillin",
  "gene_symbol": "PXN",
  "gene": "UniProtKB:P49023",
  "term_id": "GO:0005925"
}